{
  "gene": "UniProtKB:Q9ULX3",
  "gene_symbol": "NOB1",
  "gene_name": "RNA-binding protein NOB1",
  "term_label": "RNA endonuclease activity",
  "term_id": "GO:0004521"
}